{
  "term_id": "GO:0005856",
  "gene_symbol": "DYRK3",
  "gene": "UniProtKB:O43781",
  "gene_name": "Dual specificity tyrosine-phosphorylation-regulated kinase 3",
  "term_label": "cytoskeleton"
}